C-X-C chemokine binding [GO:0019958] (MF) Sources: GOC:ai Relationships: is a type of chemokine binding [GO:0019956] Definition: Binding to a C-X-C chemokine; C-X-C chemokines have a single amino acid between the first two cysteines of the characteristic four cysteine motif. Subtypes: interleukin-8 binding [GO:0019959]